{
  "gene_name": "Testis-specific Y-encoded-like protein 5",
  "term_id": "GO:0005634",
  "term_label": "nucleus",
  "gene": "UniProtKB:Q86VY4",
  "gene_symbol": "TSPYL5"
}